positive regulation of renal sodium excretion by pressure natriuresis [GO:0035819] (biological process) Relationships: is a type of pressure natriuresis [GO:0003095]; is a type of GO:0035815 Definition: An increase in the amount of sodium excreted in urine over a unit of time, as a result of pressure natriuresis. Also known as: natriuresis resulting from pressure natriuresis Sources: GOC:mtg_25march11, GOC:yaf